{
  "gene": "UniProtKB:Q9P2G3",
  "term_id": "UNKNOWN:0002",
  "gene_symbol": "KLHL14",
  "gene_name": "Kelch-like protein 14",
  "term_label": "Unknown biological process"
}